{
  "term_id": "GO:0000103",
  "gene": "UniProtKB:O43252",
  "term_label": "sulfate assimilation",
  "gene_symbol": "PAPSS1",
  "gene_name": "Bifunctional 3'-phosphoadenosine 5'-phosphosulfate synthase 1"
}